{
  "term_label": "dense core granule priming",
  "gene": "UniProtKB:Q8NB66",
  "gene_name": "Protein unc-13 homolog C",
  "gene_symbol": "UNC13C",
  "term_id": "GO:0061789"
}